{
  "gene_symbol": "SEC24D",
  "term_id": "GO:0030127",
  "gene": "UniProtKB:O94855",
  "term_label": "COPII vesicle coat",
  "gene_name": "Protein transport protein Sec24D"
}